{
  "term_id": "GO:0003950",
  "gene_name": "Protein mono-ADP-ribosyltransferase PARP11",
  "gene": "UniProtKB:Q9NR21",
  "term_label": "NAD+ poly-ADP-ribosyltransferase activity",
  "gene_symbol": "PARP11"
}